mesonephric epithelium development [GO:0072163] (biological process) Definition: The process whose specific outcome is the progression of an epithelium in the mesonephros over time, from its formation to the mature structure. An epithelium is a tissue that covers the internal or external surfaces of an anatomical structure. Subtypes: GO:0061241, GO:0072164 Sources: GOC:mtg_kidney_jan10 Relationships: is a type of GO:0072073; is part of GO:0001823